{
  "term_label": "L-serine catabolic process",
  "gene_symbol": "SDS",
  "term_id": "GO:0006565",
  "gene": "UniProtKB:P20132",
  "gene_name": "L-serine dehydratase_L-threonine deaminase"
}